{
  "gene_name": "Immunoglobulin kappa variable 3D-20",
  "gene_symbol": "IGKV3D-20",
  "term_id": "GO:0019814",
  "term_label": "immunoglobulin complex",
  "gene": "UniProtKB:A0A0C4DH25"
}